telomere-telomerase complex assembly [GO:1905324] (biological process) References: PMID:26305931 Sources: GOC:TermGenie, GO_REF:0000079 Relationships: is a type of protein-DNA complex assembly [GO:0065004]; is part of GO:0032200 Definition: The aggregation, arrangement and bonding together of a set of components to form a telomere-telomerase complex. Also known as: telomere-telomerase complex formation